phosphocreatine biosynthetic process [GO:0046314] (biological process) Relationships: is a type of phosphocreatine metabolic process [GO:0006603]; is a type of phosphagen biosynthetic process [GO:0042396] Definition: The chemical reactions and pathways resulting in the formation of phosphocreatine, a phosphagen of creatine which is synthesized and broken down by creatine phosphokinase. Sources: GOC:ai Also known as: phosphocreatine anabolism, phosphocreatine biosynthesis, phosphocreatine formation, phosphocreatine synthesis